{
  "gene_symbol": "CLSTN1",
  "gene_name": "Calsyntenin-1",
  "gene": "UniProtKB:O94985",
  "term_id": "GO:0098632",
  "term_label": "cell-cell adhesion mediator activity"
}